{
  "term_label": "intracellular zinc ion homeostasis",
  "gene_symbol": "MT1DP",
  "gene_name": "Putative metallothionein MT1DP",
  "gene": "UniProtKB:A1L3X4",
  "term_id": "GO:0006882"
}